{
  "gene_symbol": "ANKRD29",
  "term_id": "UNKNOWN:0002",
  "term_label": "Unknown biological process",
  "gene": "UniProtKB:Q8N6D5",
  "gene_name": "Ankyrin repeat domain-containing protein 29"
}